{
  "term_label": "Unknown biological process",
  "gene_name": "Phosphatidylinositol-glycan biosynthesis class X protein",
  "gene": "UniProtKB:Q8TBF5",
  "term_id": "UNKNOWN:0002",
  "gene_symbol": "PIGX"
}